negative regulation of engulfment of apoptotic cell [GO:1901075] (biological process) References: PMID:19402756 Sources: GO:kmv, GOC:TermGenie Definition: Any process that stops, prevents or reduces the frequency, rate or extent of engulfment of apoptotic cell. Also known as: down regulation of engulfment of apoptotic cell, down regulation of engulfment of apoptotic cell corpse, down regulation of engulfment of cell corpse, down-regulation of engulfment of apoptotic cell, down-regulation of engulfment of apoptotic cell corpse, down-regulation of engulfment of cell corpse, downregulation of engulfment of apoptotic cell, downregulation of engulfment of apoptotic cell corpse, downregulation of engulfment of cell corpse, negative regulation of engulfment of apoptotic cell corpse, negative regulation of engulfment of cell corpse, inhibition of engulfment of apoptotic cell, inhibition of engulfment of apoptotic cell corpse, inhibition of engulfment of cell corpse Relationships: is a type of negative regulation of phagocytosis, engulfment [GO:0060101]; is a type of GO:1901074; is a type of negative regulation of apoptotic cell clearance [GO:2000426]; negatively regulates engulfment of apoptotic cell [GO:0043652]